ciliary necklace assembly [GO:1905352] (biological process) References: PMID:20399632, PMID:6409906 Sources: GOC:TermGenie, GOC:cilia, GO_REF:0000079 Relationships: is a type of protein-containing complex assembly [GO:0065003] Also known as: cilial necklace assembly, cilial necklace formation, ciliary necklace formation, cilium necklace assembly, cilium necklace formation Definition: The aggregation, arrangement and bonding together of a set of components to form a ciliary necklace.